core TFIIH complex portion of NEF3 complex [GO:0000440] (cellular component) Definition: The core TFIIH complex when it is part of the nucleotide-excision repair factor 3 (NEF3). References: PMID:14500720, PMID:22308316, PMID:22572993, PMID:7813015 Sources: GOC:ew, GOC:krc Also known as: SSL2-core TFIIH complex portion of NEF3 complex Relationships: is_a transcription factor TFIIH core complex [GO:0000439]; is part of nucleotide-excision repair factor 3 complex [GO:0000112]